{
  "gene_name": "Flotillin-1",
  "term_id": "GO:0016600",
  "term_label": "flotillin complex",
  "gene_symbol": "FLOT1",
  "gene": "UniProtKB:O75955"
}